oxalate oxidase activity [GO:0050162] (molecular function) Relationships: is a type of GO:0016623 Definition: Catalysis of the reaction: 2 H+ + O2 + oxalate = 2 CO2 + H2O2. Sources: RHEA:21880 Also known as: aero-oxalo dehydrogenase activity, oxalate:oxygen oxidoreductase activity, oxalic acid oxidase activity